{
  "gene": "UniProtKB:Q8WWB5",
  "gene_symbol": "PIH1D2",
  "term_id": "GO:0097255",
  "term_label": "R2TP complex",
  "gene_name": "PIH1 domain-containing protein 2"
}